{
  "gene_name": "F-box only protein 25",
  "gene": "UniProtKB:Q8TCJ0",
  "gene_symbol": "FBXO25",
  "term_id": "GO:0019005",
  "term_label": "SCF ubiquitin ligase complex"
}